{
  "gene_name": "Serine incorporator 4",
  "term_id": "UNKNOWN:0002",
  "term_label": "Unknown biological process",
  "gene_symbol": "SERINC4",
  "gene": "UniProtKB:A6NH21"
}